stomach smooth muscle contraction [GO:0120063] (biological process) References: PMID:15890336 Sources: GOC:sl Relationships: is_a gastro-intestinal system smooth muscle contraction [GO:0014831] Subtypes: distal stomach smooth muscle contraction [GO:0014828], proximal stomach smooth muscle contraction [GO:0014847] Definition: A process in which force is generated within gastric smooth muscle tissue, resulting in a change in muscle geometry. This process occurs throughout the length of the stomach.